{
  "gene": "UniProtKB:Q9NS91",
  "term_label": "nucleus",
  "gene_name": "E3 ubiquitin-protein ligase RAD18",
  "term_id": "GO:0005634",
  "gene_symbol": "RAD18"
}